{
  "gene_name": "NACHT, LRR and PYD domains-containing protein 10",
  "gene_symbol": "NLRP10",
  "term_label": "cytoplasm",
  "term_id": "GO:0005737",
  "gene": "UniProtKB:Q86W26"
}